{
  "gene_symbol": "QARS1",
  "term_label": "cytosol",
  "gene": "UniProtKB:P47897",
  "term_id": "GO:0005829",
  "gene_name": "Glutamine--tRNA ligase"
}